regulation of transmembrane transporter activity [GO:0022898] (BP) Definition: Any process that modulates the frequency, rate or extent of transmembrane transporter activity. Sources: GOC:dph, GOC:mtg_cardio, GOC:mtg_transport Relationships: is a type of regulation of transmembrane transport [GO:0034762]; is a type of GO:0065009; regulates transmembrane transporter activity [GO:0022857] Subtypes: GO:0032413, positive regulation of ion transmembrane transporter activity [GO:0032414], regulation of ryanodine-sensitive calcium-release channel activity [GO:0060314], regulation of store-operated calcium channel activity [GO:1901339], GO:1901385, GO:1901894, regulation of cyclic nucleotide-gated ion channel activity [GO:1902159], regulation of delayed rectifier potassium channel activity [GO:1902259], regulation of water channel activity [GO:1902427], regulation of potassium:proton exchanging ATPase activity [GO:1904451], regulation of cytochrome-c oxidase activity [GO:1904959], positive regulation of oxidative phosphorylation uncoupler activity [GO:2000277], regulation of NMDA receptor activity [GO:2000310], regulation of AMPA receptor activity [GO:2000311], GO:2000649